{
  "term_label": "DNA polymerase binding",
  "gene_name": "Fanconi anemia group D2 protein",
  "gene": "UniProtKB:Q9BXW9",
  "term_id": "GO:0070182",
  "gene_symbol": "FANCD2"
}